eye pigment biosynthetic process [GO:0006726] (biological process) Subtypes: ommochrome biosynthetic process [GO:0006727], rhodopsin biosynthetic process [GO:0016063] Also known as: eye pigment anabolism, eye pigment biosynthesis, eye pigment formation, eye pigment synthesis Definition: The chemical reactions and pathways resulting in the formation of eye pigments, any general or particular coloring matter in living organisms, found or utilized in the eye. Sources: GOC:ai Relationships: is a type of eye pigment metabolic process [GO:0042441]; is a type of pigment biosynthetic process [GO:0046148]